{
  "term_id": "UNKNOWN:0002",
  "gene_symbol": "C12orf54",
  "term_label": "Unknown biological process",
  "gene": "UniProtKB:Q6X4T0",
  "gene_name": "Uncharacterized protein C12orf54"
}